{
  "term_label": "nucleus",
  "gene_symbol": "RAI1",
  "gene_name": "Retinoic acid-induced protein 1",
  "term_id": "GO:0005634",
  "gene": "UniProtKB:Q7Z5J4"
}